{
  "gene_symbol": "CRTAP",
  "term_label": "collagen fibril organization",
  "term_id": "GO:0030199",
  "gene_name": "Cartilage-associated protein",
  "gene": "UniProtKB:O75718"
}